{
  "term_label": "tRNA-uridine aminocarboxypropyltransferase activity",
  "term_id": "GO:0016432",
  "gene_symbol": "DTWD1",
  "gene": "UniProtKB:Q8N5C7",
  "gene_name": "tRNA-uridine aminocarboxypropyltransferase 1"
}